{
  "term_id": "UNKNOWN:0002",
  "gene": "UniProtKB:P20933",
  "term_label": "Unknown biological process",
  "gene_name": "N(4)-(beta-N-acetylglucosaminyl)-L-asparaginase",
  "gene_symbol": "AGA"
}